{
  "gene": "UniProtKB:Q9NS40",
  "term_label": "regulation of membrane potential",
  "term_id": "GO:0042391",
  "gene_name": "Potassium voltage-gated channel subfamily H member 7",
  "gene_symbol": "KCNH7"
}